{
  "term_label": "keratinization",
  "gene_name": "Keratin, type II cytoskeletal 3",
  "gene": "UniProtKB:P12035",
  "term_id": "GO:0031424",
  "gene_symbol": "KRT3"
}